{
  "gene_symbol": "MEIS1",
  "term_label": "DNA-binding transcription activator activity, RNA polymerase II-specific",
  "term_id": "GO:0001228",
  "gene": "UniProtKB:O00470",
  "gene_name": "Homeobox protein Meis1"
}